{
  "term_id": "GO:0000981",
  "gene_symbol": "ZNF768",
  "gene_name": "Zinc finger protein 768",
  "term_label": "DNA-binding transcription factor activity, RNA polymerase II-specific",
  "gene": "UniProtKB:Q9H5H4"
}